{
  "gene": "UniProtKB:Q6YFQ2",
  "gene_name": "Cytochrome c oxidase subunit 6B2",
  "term_id": "UNKNOWN:0001",
  "gene_symbol": "COX6B2",
  "term_label": "Unknown molecular function"
}